pole plasm protein localization [GO:0007318] (biological process) Also known as: establishment and maintenance of pole plasm protein localization, oocyte pole plasm protein localization, pole plasm protein localisation Sources: GOC:ai Relationships: is a type of intracellular protein localization [GO:0008104]; is part of pole plasm assembly [GO:0007315] Definition: Any process in which a protein is transported to, or maintained in, the oocyte pole plasm. An example of this is found in Drosophila melanogaster.